alphaIIb-beta3 integrin-ICAM-4 complex [GO:0071113] (cellular component) Also known as: ITGAIIb-ITGB3-ICAM4 complex Relationships: is a type of plasma membrane protein complex [GO:0098797] References: PMID:12477717 Definition: A protein complex that consists of an alphaIIb-beta3 integrin complex bound to the cell adhesion molecule ICAM-4.